regulation of microtubule-based process [GO:0032886] (biological process) Relationships: is a type of regulation of cellular process [GO:0050794]; regulates microtubule-based process [GO:0007017] Subtypes: regulation of spindle elongation [GO:0032887], GO:0046605, regulation of microtubule-based movement [GO:0060632], regulation of microtubule cytoskeleton organization [GO:0070507] Sources: GOC:mah Definition: Any process that modulates the frequency, rate or extent of any cellular process that depends upon or alters the microtubule cytoskeleton.